{
  "gene": "UniProtKB:O43290",
  "gene_name": "U4_U6.U5 tri-snRNP-associated protein 1",
  "term_label": "maturation of 5S rRNA",
  "term_id": "GO:0000481",
  "gene_symbol": "SART1"
}